{
  "gene": "UniProtKB:Q8NCR6",
  "gene_symbol": "SMRP1",
  "term_label": "manchette",
  "term_id": "GO:0002177",
  "gene_name": "Spermatid-specific manchette-related protein 1"
}